{
  "gene_symbol": "COLEC11",
  "term_label": "Unknown molecular function",
  "term_id": "UNKNOWN:0001",
  "gene": "UniProtKB:Q9BWP8",
  "gene_name": "Collectin-11"
}